kinetochore binding [GO:0043515] (MF) Relationships: is a type of GO:0005488 Sources: GOC:jl Definition: Binding to a kinetochore, a proteinaceous structure on a condensed chromosome, beside the centromere, to which the spindle fibers are attached.